D-allose catabolic process [GO:0019316] (biological process) Sources: GOC:ai, GOC:jsg, GOC:mah Also known as: D-allose breakdown, D-allose catabolism, D-allose degradation Definition: The chemical reactions and pathways resulting in the breakdown of D-allose, the D-enantiomer of allo-hexose, an aldohexose similar to glucose. Relationships: is a type of hexose catabolic process [GO:0019320]